{
  "term_label": "retinal rod cell development",
  "gene_name": "Protein fantom",
  "term_id": "GO:0046548",
  "gene_symbol": "RPGRIP1L",
  "gene": "UniProtKB:Q68CZ1"
}